{
  "gene": "UniProtKB:Q7Z591",
  "term_id": "GO:0005813",
  "gene_symbol": "AKNA",
  "gene_name": "Microtubule organization protein AKNA",
  "term_label": "centrosome"
}